{
  "gene_name": "Elongation factor 2",
  "gene": "UniProtKB:P13639",
  "gene_symbol": "EEF2",
  "term_label": "GTPase activity",
  "term_id": "GO:0003924"
}